fumarate transmembrane transporter activity [GO:0015138] (MF) Definition: Enables the transfer of fumarate from one side of a membrane to the other. Fumarate is a key intermediate in metabolism and is formed in the TCA cycle from succinate and converted into malate. Subtypes: succinate:fumarate antiporter activity [GO:0005469], GO:0062057 Also known as: dicarboxylate (succinate/fumarate/malate) antiporter activity Relationships: is a type of dicarboxylic acid transmembrane transporter activity [GO:0005310]; is a type of C4-dicarboxylate transmembrane transporter activity [GO:0015556]; is part of GO:0015741 Sources: GOC:ai